{
  "gene": "UniProtKB:Q99743",
  "gene_symbol": "NPAS2",
  "term_label": "regulation of transcription by RNA polymerase II",
  "term_id": "GO:0006357",
  "gene_name": "Neuronal PAS domain-containing protein 2"
}